negative regulation of ribosomal large subunit export from nucleus [GO:2000204] (biological process) Definition: Any process that stops, prevents, or reduces the frequency, rate or extent of ribosomal large subunit export from nucleus. Sources: GOC:mah Also known as: negative regulation of ribosomal large subunit export from cell nucleus, negative regulation of ribosomal large subunit export out of nucleus, negative regulation of ribosomal large subunit transport from nucleus to cytoplasm, negative regulation of ribosomal large subunit-nucleus export, negative regulation of 50S ribosomal subunit export from nucleus, negative regulation of 60S ribosomal subunit export from nucleus Relationships: is a type of negative regulation of ribosomal subunit export from nucleus [GO:2000201]; is a type of regulation of ribosomal large subunit export from nucleus [GO:2000203]; negatively regulates ribosomal large subunit export from nucleus [GO:0000055]